interstitial hexagonal collagen network [GO:0098646] (CC) Definition: A hexagonal shaped collagen network formed by collagen type X trimer, mostly found in the cartilage hyaline matrix, which located in the interstitial area. References: PMID:21421911, PMID:34948124 Also known as: collagen hexagonal network Relationships: is a type of GO:0098645; is part of collagenous component of interstitial matrix [GO:0140152]